beta-alanyl amine synthase activity [GO:0003833] (MF) Definition: Catalysis of the synthesis of beta-alanyl amine conjugate from a precursor biogenic amine, such as dopamine or histamine. Also known as: N-beta-alanyl dopamine synthetase activity, NBAD transferase activity, beta-alanyl-dopamine synthase activity Relationships: is a type of ligase activity, forming carbon-nitrogen bonds [GO:0016879] References: PMID:12900414, PMID:12957543, PMID:25229196 Sources: GOC:bf